{
  "gene_symbol": "SMIM34",
  "gene_name": "Small integral membrane protein 34",
  "term_id": "UNKNOWN:0003",
  "gene": "UniProtKB:A8MWV9",
  "term_label": "Unknown cellular component"
}